small intestinal transit [GO:0120055] (biological process) References: PMID:15890336 Sources: GOC:sl Definition: Migration of ingested material along the length of the small intestine. Relationships: is a type of intestinal motility [GO:0120054] Also known as: small bowel transit, small intestine transit Regulation: regulated by regulation of small intestinal transit [GO:0120057]; positively regulated by GO:0120058; negatively regulated by negative regulation of small intestinal transit [GO:0120059]